{
  "term_label": "plasma membrane",
  "term_id": "GO:0005886",
  "gene_name": "B-cell differentiation antigen CD72",
  "gene": "UniProtKB:P21854",
  "gene_symbol": "CD72"
}